{
  "term_id": "UNKNOWN:0003",
  "gene_name": "Intermembrane lipid transfer protein VPS13A",
  "term_label": "Unknown cellular component",
  "gene": "UniProtKB:Q96RL7",
  "gene_symbol": "VPS13A"
}